{
  "gene_symbol": "NECAP2",
  "term_label": "Unknown molecular function",
  "term_id": "UNKNOWN:0001",
  "gene": "UniProtKB:Q9NVZ3",
  "gene_name": "Adaptin ear-binding coat-associated protein 2"
}